brown fat cell differentiation [GO:0050873] (biological process) Relationships: is a type of GO:0045444 Also known as: brown adipocyte cell differentiation, brown adipocyte differentiation Regulation: RO_0002211 by regulation of brown fat cell differentiation [GO:0090335]; positively regulated by GO:0090336; negatively regulated by GO:1903444 Definition: The process in which a relatively unspecialized cell acquires specialized features of a brown adipocyte, an animal connective tissue cell involved in adaptive thermogenesis. Brown adipocytes contain multiple small droplets of triglycerides and a high number of mitochondria. References: PMID:12588810